{
  "gene": "UniProtKB:Q96M02",
  "gene_symbol": "C10orf90",
  "term_label": "ubiquitin protein ligase activity",
  "gene_name": "(E2-independent) E3 ubiquitin-conjugating enzyme FATS",
  "term_id": "GO:0061630"
}